{
  "gene_name": "Microcephalin",
  "term_id": "UNKNOWN:0001",
  "gene_symbol": "MCPH1",
  "gene": "UniProtKB:Q8NEM0",
  "term_label": "Unknown molecular function"
}